{
  "gene_name": "Protein Wnt-9a",
  "term_label": "cell fate commitment",
  "gene_symbol": "WNT9A",
  "gene": "UniProtKB:O14904",
  "term_id": "GO:0045165"
}